catechol catabolic process, meta-cleavage [GO:0019616] (biological process) Definition: The chemical reactions and pathways resulting in the breakdown of catechol via the meta-cleavage pathway, in which the catechol aromatic ring is broken between a hydroxylated carbon atom and an adjacent unsubstituted carbon atom. References: PMID:7765833 Sources: GOC:jl Also known as: catechol breakdown, meta-cleavage, catechol degradation, meta-cleavage Relationships: is a type of catechol-containing compound catabolic process [GO:0019614]